{
  "gene_name": "Ubiquitin-like modifier-activating enzyme 1",
  "gene": "UniProtKB:P22314",
  "term_id": "GO:0016567",
  "gene_symbol": "UBA1",
  "term_label": "protein ubiquitination"
}